{
  "term_id": "UNKNOWN:0002",
  "gene_name": "Olfactory receptor 8K3",
  "gene_symbol": "OR8K3",
  "term_label": "Unknown biological process",
  "gene": "UniProtKB:Q8NH51"
}